cirsimaritin 4'-O-methyltransferase activity [GO:0102625] (MF) Definition: Catalysis of the reaction: cirsimaritin + S-adenosyl-L-methionine = H+ + S-adenosyl-L-homocysteine + salvigenin. Sources: RHEA:73251 Relationships: is_a GO:0008168